{
  "term_id": "UNKNOWN:0001",
  "term_label": "Unknown molecular function",
  "gene": "UniProtKB:Q8NBT0",
  "gene_symbol": "POC1A",
  "gene_name": "POC1 centriolar protein homolog A"
}